butanediol biosynthetic process [GO:0034079] (biological process) Also known as: butanediol anabolism, butanediol biosynthesis, butanediol fermentation, butanediol formation, butanediol synthesis, butylene glycol biosynthesis, butylene glycol biosynthetic process, pyruvate fermentation to butanediol, glycolytic fermentation to butanediol Relationships: is_a pyruvate fermentation [GO:0019660]; is a type of butanediol metabolic process [GO:0034077]; is a type of glycol biosynthetic process [GO:0042845]; is a type of secondary alcohol biosynthetic process [GO:1902653]; has part GO:0000721; has part GO:0003984; has part acetolactate decarboxylase activity [GO:0047605]; has part diacetyl reductase ((R)-acetoin forming) (NAD+) activity [GO:0052587] Definition: The chemical reactions and pathways resulting in the formation of butanediol; the biologically relevant isomer is 2,3-butanediol, CH3CH(OH)CH(OH)CH3. Sources: GOC:mah, ISBN:0911910123, MetaCyc:P125-PWY